{
  "gene_symbol": "KCTD21",
  "term_label": "cullin family protein binding",
  "term_id": "GO:0097602",
  "gene_name": "BTB_POZ domain-containing protein KCTD21",
  "gene": "UniProtKB:Q4G0X4"
}